{
  "gene": "UniProtKB:Q7L0X0",
  "term_id": "GO:0034142",
  "term_label": "toll-like receptor 4 signaling pathway",
  "gene_symbol": "TRIL",
  "gene_name": "TLR4 interactor with leucine rich repeats"
}